{
  "term_id": "GO:0005096",
  "term_label": "GTPase activator activity",
  "gene_symbol": "ARHGAP19",
  "gene": "UniProtKB:Q14CB8",
  "gene_name": "Rho GTPase-activating protein 19"
}